neutrophil extracellular trap [GO:0140644] (cellular component) Definition: Extracellular microbicidal structure composed of nuclear chromatin, histones and granular antimicrobial proteins. Histones and several neutrophil granule proteins associated with the DNA framework damage entrapped microorganisms. Also known as: NET Relationships: is a type of extracellular membraneless organelle [GO:0043264] References: PMID:31172493